{
  "gene_name": "Heat shock factor 2-binding protein",
  "gene": "UniProtKB:O75031",
  "term_label": "cytosol",
  "gene_symbol": "HSF2BP",
  "term_id": "GO:0005829"
}